{
  "gene": "UniProtKB:Q8NGW6",
  "gene_name": "Olfactory receptor 6K6",
  "term_label": "olfactory receptor activity",
  "gene_symbol": "OR6K6",
  "term_id": "GO:0004984"
}